{
  "gene_name": "Junctional adhesion molecule A",
  "gene": "UniProtKB:Q9Y624",
  "term_label": "Unknown molecular function",
  "gene_symbol": "F11R",
  "term_id": "UNKNOWN:0001"
}